{
  "gene_name": "Sorting nexin-6",
  "term_label": "endosome",
  "term_id": "GO:0005768",
  "gene_symbol": "SNX6",
  "gene": "UniProtKB:Q9UNH7"
}